{
  "gene_symbol": "SLC16A2",
  "term_id": "GO:0070327",
  "gene_name": "Monocarboxylate transporter 8",
  "term_label": "thyroid hormone transport",
  "gene": "UniProtKB:P36021"
}